{
  "gene_symbol": "CFAP61",
  "term_id": "UNKNOWN:0001",
  "gene": "UniProtKB:Q8NHU2",
  "gene_name": "Cilia- and flagella-associated protein 61",
  "term_label": "Unknown molecular function"
}